{
  "term_id": "GO:0000977",
  "term_label": "RNA polymerase II transcription regulatory region sequence-specific DNA binding",
  "gene_symbol": "TCF23",
  "gene_name": "Transcription factor 23",
  "gene": "UniProtKB:Q7RTU1"
}